negative regulation of platelet activation [GO:0010544] (biological process) Definition: Any process that decreases the rate or frequency of platelet activation. Platelet activation is a series of progressive, overlapping events triggered by exposure of the platelets to subendothelial tissue. Sources: GOC:BHF, GOC:dph, GOC:tb Relationships: is a type of regulation of platelet activation [GO:0010543]; is a type of negative regulation of blood coagulation [GO:0030195]; is a type of negative regulation of cell activation [GO:0050866]; negatively regulates platelet activation [GO:0030168] Subtypes: negative regulation of platelet aggregation [GO:0090331]